{
  "gene_name": "Transmembrane protein 184B",
  "term_id": "UNKNOWN:0002",
  "term_label": "Unknown biological process",
  "gene": "UniProtKB:Q9Y519",
  "gene_symbol": "TMEM184B"
}